{
  "term_id": "GO:0007342",
  "gene_symbol": "FOLR2",
  "term_label": "fusion of sperm to egg plasma membrane involved in single fertilization",
  "gene": "UniProtKB:P14207",
  "gene_name": "Folate receptor beta"
}